virion membrane [GO:0055036] (cellular component) Relationships: is a type of virion component [GO:0044423] References: PMID:213106 Sources: GOC:jid, GOC:rph Definition: The lipid bilayer surrounding a virion.